{
  "gene_name": "Postmeiotic segregation increased 2-like protein 5",
  "term_label": "Unknown molecular function",
  "gene": "UniProtKB:A8MQ11",
  "gene_symbol": "PMS2P5",
  "term_id": "UNKNOWN:0001"
}